respiratory chain complex [GO:0098803] (cellular component) Sources: GOC:dos Definition: Any protein complex that is part of a respiratory chain. Also known as: respirasome Relationships: is a type of protein-containing complex [GO:0032991] Subtypes: cytochrome o ubiquinol oxidase complex [GO:0009319], NarGHI complex [GO:0044799], proton-transporting ATP synthase complex [GO:0045259], respiratory chain complex I [GO:0045271], respiratory chain complex II (succinate dehydrogenase) [GO:0045273], respiratory chain complex III [GO:0045275], respiratory chain complex IV [GO:0045277], fumarate reductase complex [GO:0045283]